{
  "term_label": "glycogen catabolic process",
  "term_id": "GO:0005980",
  "gene": "UniProtKB:P11216",
  "gene_symbol": "PYGB",
  "gene_name": "Glycogen phosphorylase, brain form"
}